leaf morphogenesis [GO:0009965] (biological process) Definition: The process in which the anatomical structures of the leaf are generated and organized. Subtypes: cotyledon morphogenesis [GO:0048826], GO:0060776, compound leaf morphogenesis [GO:0060777] Sources: GOC:go_curators Regulation: RO_0002211 by GO:1901371 Relationships: is a type of plant organ morphogenesis [GO:1905392]; is part of GO:0010016; is part of leaf development [GO:0048366]